{
  "term_label": "unfolded protein binding",
  "gene_name": "Cell cycle and apoptosis regulator protein 2",
  "gene_symbol": "CCAR2",
  "term_id": "GO:0051082",
  "gene": "UniProtKB:Q8N163"
}